{
  "gene_name": "Tigger transposable element-derived protein 4",
  "gene_symbol": "TIGD4",
  "gene": "UniProtKB:Q8IY51",
  "term_label": "DNA binding",
  "term_id": "GO:0003677"
}